{
  "term_label": "microtubule cytoskeleton",
  "term_id": "GO:0015630",
  "gene": "UniProtKB:Q6PGN9",
  "gene_name": "Proline_serine-rich coiled-coil protein 1",
  "gene_symbol": "PSRC1"
}